{
  "gene_symbol": "MARCOL",
  "term_id": "UNKNOWN:0001",
  "term_label": "Unknown molecular function",
  "gene_name": "MARCO-like protein",
  "gene": "UniProtKB:A0A1B0GUY1"
}